{
  "gene": "UniProtKB:Q8N474",
  "gene_name": "Secreted frizzled-related protein 1",
  "term_label": "Wnt-protein binding",
  "gene_symbol": "SFRP1",
  "term_id": "GO:0017147"
}